{
  "gene": "UniProtKB:P62888",
  "gene_name": "Large ribosomal subunit protein eL30",
  "gene_symbol": "RPL30",
  "term_id": "GO:0003723",
  "term_label": "RNA binding"
}